{
  "term_id": "GO:0031514",
  "term_label": "motile cilium",
  "gene_name": "Cation channel sperm-associated auxiliary subunit gamma",
  "gene_symbol": "CATSPERG",
  "gene": "UniProtKB:Q6ZRH7"
}